{
  "term_id": "GO:0005615",
  "term_label": "extracellular space",
  "gene_name": "Mucin-5B",
  "gene": "UniProtKB:Q9HC84",
  "gene_symbol": "MUC5B"
}